{
  "term_id": "GO:0004867",
  "term_label": "serine-type endopeptidase inhibitor activity",
  "gene_symbol": "SERPINA10",
  "gene_name": "Protein Z-dependent protease inhibitor",
  "gene": "UniProtKB:Q9UK55"
}